{
  "gene_name": "TNF receptor-associated factor 3",
  "gene": "UniProtKB:Q13114",
  "term_label": "cytoplasm",
  "gene_symbol": "TRAF3",
  "term_id": "GO:0005737"
}